{
  "term_label": "microtubule severing",
  "term_id": "GO:0051013",
  "gene": "UniProtKB:Q6PIW4",
  "gene_symbol": "FIGNL1",
  "gene_name": "Fidgetin-like protein 1"
}